{
  "term_label": "postsynaptic recycling endosome",
  "gene_symbol": "STX12",
  "gene_name": "Syntaxin-12",
  "gene": "UniProtKB:Q86Y82",
  "term_id": "GO:0098837"
}